{
  "gene": "UniProtKB:P50391",
  "gene_symbol": "NPY4R",
  "term_id": "GO:0001602",
  "gene_name": "Neuropeptide Y receptor type 4",
  "term_label": "pancreatic polypeptide receptor activity"
}